F-bar domain binding [GO:1990808] (molecular function) Definition: Binding to an F-BAR domain of a protein, a domain of about 60 residues that occurs in a wide range of cytoskeletal proteins. References: PMID:20603077 Relationships: is a type of GO:0019904